{
  "term_id": "GO:0006357",
  "gene_name": "Zinc finger protein 490",
  "gene": "UniProtKB:Q9ULM2",
  "gene_symbol": "ZNF490",
  "term_label": "regulation of transcription by RNA polymerase II"
}